{
  "gene": "UniProtKB:Q9GZT9",
  "term_label": "nucleus",
  "gene_name": "Egl nine homolog 1",
  "gene_symbol": "EGLN1",
  "term_id": "GO:0005634"
}